{
  "gene": "UniProtKB:Q16706",
  "gene_symbol": "MAN2A1",
  "gene_name": "Alpha-mannosidase 2",
  "term_id": "GO:0006491",
  "term_label": "N-glycan processing"
}